{
  "gene_name": "Glycine N-methyltransferase",
  "term_id": "GO:0042802",
  "gene_symbol": "GNMT",
  "term_label": "identical protein binding",
  "gene": "UniProtKB:Q14749"
}